peptidyl-lysine hydroxylation to 5-hydroxy-L-lysine [GO:0018395] (biological process) Definition: The hydroxylation of peptidyl-lysine to peptidyl-5-hydroxy-L-lysine. Sources: RESID:AA0028 Relationships: is a type of peptidyl-lysine hydroxylation [GO:0017185]